{
  "term_id": "GO:0004930",
  "gene": "UniProtKB:Q9BZJ7",
  "gene_name": "G-protein coupled receptor 62",
  "term_label": "G protein-coupled receptor activity",
  "gene_symbol": "GPR62"
}